FYXD domain binding [GO:0098750] (molecular function) Relationships: is_a protein domain specific binding [GO:0019904] References: PMID:10950925, PMID:16403837, PMID:18000745 Sources: GOC:dos, GOC:mr Definition: Binding to a FXYD domain.